rhodopsin kinase activity [GO:0050254] (molecular function) Definition: Catalysis of the reaction: ATP + rhodopsin = ADP + phosphorhodopsin. Also known as: rhodopsin kinase (phosphorylating) activity, GPCR kinase 1 activity, cone opsin kinase activity, opsin kinase (phosphorylating) activity, opsin kinase activity Relationships: is a type of G protein-coupled receptor kinase activity [GO:0004703] References: PMID:14654303